{
  "gene": "UniProtKB:Q9NR16",
  "term_label": "Unknown biological process",
  "term_id": "UNKNOWN:0002",
  "gene_name": "Scavenger receptor cysteine-rich type 1 protein M160",
  "gene_symbol": "CD163L1"
}